negative regulation of fibrinolysis [GO:0051918] (biological process) Definition: Any process that stops, prevents, or reduces the frequency, rate or extent of fibrinolysis, an ongoing process that solubilizes fibrin, resulting in the removal of small blood clots. Sources: GOC:ai Also known as: down regulation of fibrinolysis, down-regulation of fibrinolysis, downregulation of fibrinolysis, inhibition of fibrinolysis Relationships: is a type of positive regulation of blood coagulation [GO:0030194]; is a type of positive regulation of response to external stimulus [GO:0032103]; is a type of negative regulation of biological process [GO:0048519]; is_a regulation of fibrinolysis [GO:0051917]; negatively regulates fibrinolysis [GO:0042730]